proximal/distal pattern formation, imaginal disc [GO:0007449] (biological process) Sources: GOC:jid, ISBN:0879694238 Definition: The establishment, maintenance and elaboration of the proximal/distal axis of the imaginal disc. Imaginal disks are masses of hypodermic cells, carried by the larvae of some insects after leaving the egg, from which masses the wings and legs of the adult are subsequently formed. Relationships: is a type of GO:0007447; is a type of proximal/distal pattern formation [GO:0009954] Subtypes: wing disc proximal/distal pattern formation [GO:0007473], GO:0007479